{
  "gene": "UniProtKB:Q13324",
  "gene_name": "Corticotropin-releasing factor receptor 2",
  "term_id": "GO:0030425",
  "gene_symbol": "CRHR2",
  "term_label": "dendrite"
}